{
  "gene": "UniProtKB:Q495B1",
  "term_id": "UNKNOWN:0003",
  "term_label": "Unknown cellular component",
  "gene_symbol": "ANKDD1A",
  "gene_name": "Ankyrin repeat and death domain-containing protein 1A"
}